sphingolipid transfer activity [GO:0120016] (molecular function) Subtypes: ceramide transfer activity [GO:0120017], sphingomyelin transfer activity [GO:0140338] Definition: Removes a sphingolipid from a membrane or a monolayer lipid particle, transports it through the aqueous phase while protected in a hydrophobic pocket, and brings it to an acceptor membrane or lipid particle. Also known as: intermembrane sphingolipid transfer activity, sphingolipid carrier activity Relationships: is a type of GO:0046624; is a type of lipid transfer activity [GO:0120013]; has part GO:0046625 References: PMID:20823909, PMID:24220498, PMID:25797198 Sources: GOC:krc